{
  "term_id": "UNKNOWN:0001",
  "gene_name": "T cell receptor beta variable 6-5",
  "gene": "UniProtKB:A0A0K0K1A5",
  "term_label": "Unknown molecular function",
  "gene_symbol": "TRBV6-5"
}